response to stress [GO:0006950] (biological process) Definition: Any process that results in a change in state or activity of a cell or an organism (in terms of movement, secretion, enzyme production, gene expression, etc.) as a result of a disturbance in organismal or cellular homeostasis, usually, but not necessarily, exogenous (e.g. temperature, humidity, ionizing radiation). Relationships: is a type of response to stimulus [GO:0050896] Regulation: regulated by GO:0080134 Also known as: response to abiotic stress, response to biotic stress Sources: GOC:mah Subtypes: GO:0001666, response to ischemia [GO:0002931], muscle hypertrophy in response to stress [GO:0003299], GO:0006952, response to osmotic stress [GO:0006970], response to oxidative stress [GO:0006979], response to sterol depletion [GO:0006991], phage shock [GO:0009271], response to heat [GO:0009408], response to cold [GO:0009409], GO:0009413, response to water deprivation [GO:0009414], GO:0009611, GO:0009635, cellular response to stress [GO:0033554], GO:0033555, response to anoxia [GO:0034059], response to fluid shear stress [GO:0034405], response to isolation stress [GO:0035900], response to immobilization stress [GO:0035902], response to topologically incorrect protein [GO:0035966], response to starvation [GO:0042594], GO:0051409, GO:0051599, response to hyperoxia [GO:0055093], GO:0061771, GO:0090664, stress response to metal ion [GO:0097501], stress response to acid chemical [GO:0097532], response to psychosocial stress [GO:1990911]